gamma-tubulin complex localization to cytoplasmic side of mitotic spindle pole body [GO:0110121] (biological process) Definition: Any process in which a gamma-tubulin complex is transported to, or maintained in, a specific location at the cytoplasmic side of the mitotic spindle pole body. References: PMID:19001497 Sources: GOC:vw Relationships: is a type of gamma-tubulin complex localization to mitotic spindle pole body [GO:1990735]